{
  "gene_name": "Peptidyl-prolyl cis-trans isomerase A-like 4G",
  "term_label": "protein folding",
  "gene_symbol": "PPIAL4G",
  "term_id": "GO:0006457",
  "gene": "UniProtKB:P0DN37"
}